{
  "gene": "UniProtKB:Q711Q0",
  "gene_name": "Cardiac-enriched FHL2-interacting protein",
  "term_id": "GO:0030018",
  "term_label": "Z disc",
  "gene_symbol": "CEFIP"
}